positive regulation of corticotropin secretion [GO:0051461] (biological process) Definition: Any process that activates or increases the frequency, rate or extent of the regulated release of corticotropin hormone from a cell. Sources: GOC:ai Also known as: positive regulation of ACTH secretion, positive regulation of adrenocorticotropic hormone secretion, positive regulation of adrenocorticotropin secretion, positive regulation of adrenotropic hormone secretion, positive regulation of adrenotropin secretion, positive regulation of corticotropic hormone secretion, up regulation of adrenocorticotropin secretion, up-regulation of adrenocorticotropin secretion, upregulation of adrenocorticotropin secretion, activation of adrenocorticotropin secretion, stimulation of adrenocorticotropin secretion Relationships: is a type of positive regulation of multicellular organismal process [GO:0051240]; is a type of regulation of corticotropin secretion [GO:0051459]; is a type of positive regulation of peptide hormone secretion [GO:0090277]; positively regulates corticotropin secretion [GO:0051458]